{
  "term_id": "GO:0061630",
  "gene_symbol": "MKRN2",
  "gene_name": "E3 ubiquitin-protein ligase makorin-2",
  "gene": "UniProtKB:Q9H000",
  "term_label": "ubiquitin protein ligase activity"
}